{
  "term_label": "Unknown cellular component",
  "gene": "UniProtKB:P59990",
  "gene_name": "Keratin-associated protein 12-1",
  "term_id": "UNKNOWN:0003",
  "gene_symbol": "KRTAP12-1"
}